plasmacytoid dendritic cell activation [GO:0002270] (biological process) References: PMID:15990333, PMID:16174109 Sources: GOC:add Definition: A change in the morphology or behavior of a plasmacytoid dendritic cell resulting from exposure to an activating factor such as a cellular or soluble ligand. Subtypes: plasmacytoid dendritic cell activation involved in immune response [GO:0002271], plasmacytoid dendritic cell differentiation [GO:0002273] Relationships: is a type of leukocyte activation [GO:0045321]